angioblast cell migration from lateral mesoderm to midline [GO:0035479] (biological process) Definition: The directed movement of angioblasts from the lateral mesoderm to the midline which occurs as part of the formation of the early midline vasculature. Relationships: is_a GO:0035476 References: PMID:11861480 Sources: GOC:dgh